glyoxalase III activity [GO:0019172] (molecular function) References: PMID:21696459, PMID:7848303 Sources: GOC:mcc, RHEA:27754 Note: Note that this term was reinstated from obsolete. Also note that this enzymatic activity converts methylglyoxal to D-lactate in a single glutathione (GSH)-independent step. The other known route for this conversion is the two-step GSH-dependent pathway catalyzed by EC:4.4.1.5 (lactoylglutathione lyase) and EC:3.1.2.6 (hydroxyacylglutathione hydrolase). Also known as: (R)-lactate hydro-lyase, D-lactate dehydratase, glutathione-independent glyoxalase activity Relationships: is a type of hydro-lyase activity [GO:0016836]; is part of lactate biosynthetic process [GO:0019249]; is part of methylglyoxal catabolic process to lactate [GO:0061727] Definition: Catalysis of the reaction: methylglyoxal + H2O = D-lactate.